{
  "term_id": "UNKNOWN:0003",
  "gene_name": "Putative nucleotidyltransferase MAB21L1",
  "term_label": "Unknown cellular component",
  "gene": "UniProtKB:Q13394",
  "gene_symbol": "MAB21L1"
}